natural killer cell mediated cytotoxicity [GO:0042267] (biological process) Subtypes: natural killer cell mediated cytotoxicity directed against tumor cell target [GO:0002420] Note: Note that either or both mechanisms mentioned in the definition may be used in this process. Note that both granule release and the engagement of death receptors on target cells result in induction of apoptosis in the target cell. Regulation: regulated by GO:0042269; negatively regulated by GO:0045953; positively regulated by positive regulation of natural killer cell mediated cytotoxicity [GO:0045954] Definition: The directed killing of a target cell by a natural killer cell through the release of granules containing cytotoxic mediators or through the engagement of death receptors. Relationships: is_a leukocyte mediated cytotoxicity [GO:0001909]; is a type of GO:0002228 Sources: GOC:add, GOC:pr Also known as: NK cell mediated cell death, NK cell mediated cell killing, NK cell mediated cytotoxicity, natural killer cell mediated cell death, natural killer cell mediated cell killing, NK cell mediated cytolysis, killer activity, natural killer cell mediated cytolysis, natural killer-cell mediated cytolysis